{
  "term_label": "cytoplasm",
  "gene_symbol": "BNIPL",
  "term_id": "GO:0005737",
  "gene": "UniProtKB:Q7Z465",
  "gene_name": "Bcl-2_adenovirus E1B 19 kDa-interacting protein 2-like protein"
}